{
  "gene": "UniProtKB:A8MWX3",
  "term_label": "Unknown molecular function",
  "gene_symbol": "WASH4P",
  "gene_name": "Putative WAS protein family homolog 4",
  "term_id": "UNKNOWN:0001"
}